{
  "gene_symbol": "TEAD2",
  "gene": "UniProtKB:Q15562",
  "term_label": "regulation of transcription by RNA polymerase II",
  "gene_name": "Transcriptional enhancer factor TEF-4",
  "term_id": "GO:0006357"
}